chloroplast small ribosomal subunit [GO:0022629] (cellular component) Also known as: chloroplast ribosomal SSU complex, chloroplast ribosomal small subunit complex Definition: The small subunit of a ribosome contained within a chloroplast. Sources: GOC:mtg_sensu Relationships: is a type of GO:0000312; is part of GO:0043253